{
  "gene_symbol": "CCNP",
  "term_label": "cyclin-dependent protein kinase holoenzyme complex",
  "term_id": "GO:0000307",
  "gene": "UniProtKB:Q9H8S5",
  "gene_name": "Cyclin-P"
}